{
  "gene": "UniProtKB:Q5VUJ5",
  "term_label": "GTPase activator activity",
  "term_id": "GO:0005096",
  "gene_name": "Putative Arf-GAP with GTPase, ANK repeat and PH domain-containing protein 7",
  "gene_symbol": "AGAP7P"
}